pyrimidine deoxyribonucleoside triphosphate metabolic process [GO:0009211] (biological process) Subtypes: pyrimidine deoxyribonucleoside triphosphate biosynthetic process [GO:0009212], pyrimidine deoxyribonucleoside triphosphate catabolic process [GO:0009213], dCTP metabolic process [GO:0046065], dTTP metabolic process [GO:0046075], dUTP metabolic process [GO:0046080] Definition: The chemical reactions and pathways involving pyrimidine deoxyribonucleoside triphosphate, a compound consisting of a pyrimidine base linked to a deoxyribose sugar esterified with triphosphate on the sugar. Also known as: pyrimidine deoxyribonucleoside triphosphate metabolism Sources: GOC:go_curators, ISBN:0198506732 Relationships: is a type of pyrimidine nucleoside triphosphate metabolic process [GO:0009147]